{
  "gene_symbol": "BEND2",
  "term_label": "Unknown biological process",
  "gene": "UniProtKB:Q8NDZ0",
  "gene_name": "BEN domain-containing protein 2",
  "term_id": "UNKNOWN:0002"
}